{
  "gene_name": "Nuclear receptor ROR-beta",
  "gene_symbol": "RORB",
  "term_label": "nuclear receptor activity",
  "gene": "UniProtKB:Q92753",
  "term_id": "GO:0004879"
}